phosphoanandamide dephosphorylation [GO:0035644] (biological process) References: PMID:16938887 Sources: GOC:BHF Definition: The process of removing one or more phosphate groups from a phosphorylated anandamide. Relationships: is a type of dephosphorylation [GO:0016311]